{
  "gene": "UniProtKB:Q9NQ69",
  "gene_name": "LIM_homeobox protein Lhx9",
  "gene_symbol": "LHX9",
  "term_label": "RNA polymerase II transcription regulatory region sequence-specific DNA binding",
  "term_id": "GO:0000977"
}